male courtship behavior, proboscis-mediated licking [GO:0016546] (biological process) Definition: The process during courtship where the male fly licks the genitalia of a stationary female fly with his proboscis. An example of this is found in Drosophila melanogaster. Relationships: is a type of male courtship behavior [GO:0008049] Also known as: male courtship behaviour, proboscis-mediated licking, male courtship behavior, licking, male courtship behaviour, licking References: PMID:11092827 Sources: GOC:mtg_sensu